{
  "gene_symbol": "GEMIN5",
  "term_label": "mRNA 3'-UTR binding",
  "gene_name": "Gem-associated protein 5",
  "gene": "UniProtKB:Q8TEQ6",
  "term_id": "GO:0003730"
}